{
  "gene_symbol": "TIMELESS",
  "term_label": "DNA replication checkpoint signaling",
  "gene_name": "Protein timeless homolog",
  "term_id": "GO:0000076",
  "gene": "UniProtKB:Q9UNS1"
}